maintenance of imaginal disc-derived wing hair orientation [GO:0035321] (biological process) Definition: Ensuring that hairs in the imaginal disc-derived wing continue to point distally during development, following the initial establishment of wing hair polarity. Relationships: is a type of proximal/distal pattern formation [GO:0009954]; is part of GO:0035317 References: PMID:15501220 Sources: GOC:mtg_sensu Also known as: maintenance of wing hair orientation